mechanoreceptor differentiation [GO:0042490] (BP) Subtypes: GO:0048886, GO:0060113, mechanoreceptor differentiation involved in mechanosensory epithelium regeneration [GO:0070656] Definition: The process in which a relatively unspecialized cell acquires specialized features of a mechanoreceptor, a cell specialized to transduce mechanical stimuli and relay that information centrally in the nervous system. Sources: CL:0000199, GOC:jl Relationships: is a type of neuron differentiation [GO:0030182] Regulation: regulated by GO:0045631; negatively regulated by negative regulation of mechanoreceptor differentiation [GO:0045632]; positively regulated by positive regulation of mechanoreceptor differentiation [GO:0045633]